{
  "gene": "UniProtKB:Q8WTV0",
  "term_label": "cholesterol import",
  "gene_symbol": "SCARB1",
  "term_id": "GO:0070508",
  "gene_name": "Scavenger receptor class B member 1"
}